negative regulation of apoptosome assembly [GO:1905101] (BP) Definition: Any process that stops, prevents or reduces the frequency, rate or extent of apoptosome assembly. References: PMID:26265044 Sources: GOC:BHF, GOC:BHF_miRNA, GOC:TermGenie, GOC:bc, GO_REF:0000058 Relationships: is a type of GO:0031333; is a type of regulation of apoptosome assembly [GO:1905100]; is a type of GO:2001234; RO_0002212 apoptosome assembly [GO:0097314] Also known as: down regulation of apoptosome assembly, down regulation of apoptosome formation, down-regulation of apoptosome assembly, down-regulation of apoptosome formation, downregulation of apoptosome assembly, downregulation of apoptosome formation, negative regulation of apoptosome formation, inhibition of apoptosome assembly, inhibition of apoptosome formation